{
  "gene_symbol": "PLCH2",
  "term_label": "phosphatidylinositol metabolic process",
  "gene_name": "1-phosphatidylinositol 4,5-bisphosphate phosphodiesterase eta-2",
  "gene": "UniProtKB:O75038",
  "term_id": "GO:0046488"
}